{
  "term_id": "GO:0018279",
  "gene_symbol": "UGGT1",
  "term_label": "protein N-linked glycosylation via asparagine",
  "gene": "UniProtKB:Q9NYU2",
  "gene_name": "UDP-glucose:glycoprotein glucosyltransferase 1"
}